{
  "term_id": "GO:0006974",
  "gene_name": "ADP-ribose glycohydrolase OARD1",
  "term_label": "DNA damage response",
  "gene": "UniProtKB:Q9Y530",
  "gene_symbol": "OARD1"
}